{
  "gene": "UniProtKB:Q8TE58",
  "gene_symbol": "ADAMTS15",
  "term_label": "extracellular matrix organization",
  "term_id": "GO:0030198",
  "gene_name": "A disintegrin and metalloproteinase with thrombospondin motifs 15"
}